{
  "term_label": "Unknown molecular function",
  "gene_symbol": "PAQR4",
  "gene": "UniProtKB:Q8N4S7",
  "gene_name": "Progestin and adipoQ receptor family member 4",
  "term_id": "UNKNOWN:0001"
}